{
  "term_id": "UNKNOWN:0001",
  "term_label": "Unknown molecular function",
  "gene": "UniProtKB:Q96IZ2",
  "gene_symbol": "ADTRP",
  "gene_name": "Androgen-dependent TFPI-regulating protein"
}